hexose phosphate transmembrane transporter activity [GO:0015119] (molecular function) Definition: Enables the transfer of hexose phosphate from one side of a membrane to the other. Hexose phosphates is any of a group of monophosphorylated aldoses with a chain of six carbon atoms in the molecule. Sources: GOC:ai, GOC:mtg_transport, ISBN:0815340729 Relationships: is a type of organophosphate ester transmembrane transporter activity [GO:0015605]; is a type of carbohydrate derivative transmembrane transporter activity [GO:1901505]; BFO_0000050 hexose phosphate transport [GO:0015712] Subtypes: glucose-6-phosphate transmembrane transporter activity [GO:0015152], GO:0015526